{
  "term_label": "cytosol",
  "gene_symbol": "PASK",
  "gene_name": "PAS domain-containing serine_threonine-protein kinase",
  "gene": "UniProtKB:Q96RG2",
  "term_id": "GO:0005829"
}